{
  "term_id": "GO:0005634",
  "gene_symbol": "HIVEP2",
  "gene": "UniProtKB:P31629",
  "term_label": "nucleus",
  "gene_name": "Transcription factor HIVEP2"
}